{
  "gene": "UniProtKB:Q96PM9",
  "term_id": "GO:0010609",
  "gene_symbol": "ZNF385A",
  "gene_name": "Zinc finger protein 385A",
  "term_label": "mRNA localization resulting in post-transcriptional regulation of gene expression"
}